{
  "gene_symbol": "FAM227B",
  "gene": "UniProtKB:Q96M60",
  "term_label": "Unknown biological process",
  "term_id": "UNKNOWN:0002",
  "gene_name": "Protein FAM227B"
}